{
  "term_label": "protein sumoylation",
  "gene_symbol": "SAE1",
  "gene_name": "SUMO-activating enzyme subunit 1",
  "gene": "UniProtKB:Q9UBE0",
  "term_id": "GO:0016925"
}